7,8-dihydroxykynurenate 8,8a-dioxygenase activity [GO:0047069] (molecular function) Sources: EC:1.13.11.10, RHEA:23400 Relationships: is a type of oxidoreductase activity, acting on single donors with incorporation of molecular oxygen, incorporation of two atoms of oxygen [GO:0016702] Definition: Catalysis of the reaction: 7,8-dihydroxykynurenate + O2 = 5-(3-carboxylato-3-oxoprop-1-en-1-yl)-4,6-dihydroxypyridine-2-carboxylate + H+. Also known as: 7,8-dihydroxykynurenate 8,8alpha-dioxygenase activity, 7,8-dihydroxykynurenate oxygenase activity, 7,8-dihydroxykynurenate:oxygen 8,8a-oxidoreductase (decyclizing), 7,8-dihydroxykynurenate:oxygen 8,8alpha-oxidoreductase (decyclizing)